positive regulation of natural killer cell differentiation [GO:0032825] (biological process) Sources: GOC:mah Note: Note that immunologists typically use the word 'development' to refer to cells of B or T cell lineages undergoing the process that GO describes as 'cell differentiation'. Subtypes: positive regulation of natural killer cell differentiation involved in immune response [GO:0032828] Also known as: positive regulation of NK cell differentiation, up regulation of natural killer cell differentiation, up-regulation of natural killer cell differentiation, upregulation of natural killer cell differentiation, activation of natural killer cell differentiation, stimulation of natural killer cell differentiation, positive regulation of natural killer cell development Definition: Any process that activates or increases the frequency, rate or extent of natural killer cell differentiation. Relationships: is a type of positive regulation of natural killer cell activation [GO:0032816]; is a type of GO:0032823; is a type of positive regulation of lymphocyte differentiation [GO:0045621]; positively regulates natural killer cell differentiation [GO:0001779]